cell migration involved in coronary angiogenesis [GO:0060981] (BP) Sources: GOC:mtg_heart Definition: The orderly movement of a cell from one site to another that will contribute to the formation of new blood vessels in the heart from pre-existing blood vessels. Relationships: is a type of cell migration involved in heart development [GO:0060973]; is part of angiogenesis involved in coronary vascular morphogenesis [GO:0060978]